endocytic targeting sequence binding [GO:0089710] (molecular function) References: PMID:8918456 Relationships: is_a GO:0005515 Definition: Binding to a endocytic signal sequence, a specific peptide sequence, of 4-6 amino acids with an essential tyrosine (Y), found on cytoplasmic tails of some cell surface membrane proteins, which directs internalization by clathrin-coated pits.